{
  "gene_symbol": "ZNF598",
  "gene": "UniProtKB:Q86UK7",
  "term_id": "GO:0043022",
  "term_label": "ribosome binding",
  "gene_name": "E3 ubiquitin-protein ligase ZNF598"
}